{
  "gene_name": "RING-type domain-containing protein",
  "term_label": "Unknown cellular component",
  "gene_symbol": "RNF228",
  "term_id": "UNKNOWN:0003",
  "gene": "UniProtKB:A0A7I2V3R4"
}